{
  "term_id": "UNKNOWN:0002",
  "term_label": "Unknown biological process",
  "gene_symbol": "CD8B",
  "gene_name": "T-cell surface glycoprotein CD8 beta chain",
  "gene": "UniProtKB:P10966"
}